{
  "term_id": "GO:0003834",
  "gene": "UniProtKB:Q16518",
  "gene_symbol": "RPE65",
  "gene_name": "Retinoid isomerohydrolase",
  "term_label": "beta-carotene 15,15'-dioxygenase activity"
}